regulation of coenzyme A biosynthetic process [GO:0080020] (biological process) Relationships: is a type of regulation of biosynthetic process [GO:0009889]; is a type of regulation of nucleobase-containing compound metabolic process [GO:0019219]; is a type of regulation of amide metabolic process [GO:0034248]; is a type of regulation of sulfur metabolic process [GO:0042762]; is a type of GO:0051174; is a type of GO:0062012; regulates coenzyme A biosynthetic process [GO:0015937] Definition: Any process that modulates the frequency, rate or extent of the chemical reactions and pathways involving coenzyme A. References: PMID:18621975